{
  "term_label": "cytoplasmic side of plasma membrane",
  "gene_symbol": "RGS1",
  "gene_name": "Regulator of G-protein signaling 1",
  "gene": "UniProtKB:Q08116",
  "term_id": "GO:0009898"
}